{
  "term_id": "GO:0003723",
  "gene_symbol": "MYEF2",
  "term_label": "RNA binding",
  "gene_name": "Myelin expression factor 2",
  "gene": "UniProtKB:Q9P2K5"
}